{
  "term_id": "GO:0048242",
  "term_label": "epinephrine secretion",
  "gene_symbol": "VIP",
  "gene_name": "VIP peptides",
  "gene": "UniProtKB:P01282"
}